proteaphagy [GO:0061816] (biological process) Relationships: is a type of macroautophagy [GO:0016236] Definition: The selective degradation of proteasomes by macroautophagy. References: PMID:26670610, PMID:27477278 Sources: GOC:dph, GOC:se